{
  "gene": "UniProtKB:P23246",
  "term_label": "regulation of DNA-templated transcription",
  "gene_symbol": "SFPQ",
  "term_id": "GO:0006355",
  "gene_name": "Splicing factor, proline- and glutamine-rich"
}